{
  "gene_symbol": "ULK2",
  "term_label": "reticulophagy",
  "term_id": "GO:0061709",
  "gene_name": "Serine_threonine-protein kinase ULK2",
  "gene": "UniProtKB:Q8IYT8"
}